{
  "gene_name": "Myosin-IIIa",
  "term_id": "GO:0032426",
  "gene_symbol": "MYO3A",
  "gene": "UniProtKB:Q8NEV4",
  "term_label": "stereocilium tip"
}